{
  "term_label": "antibacterial humoral response",
  "gene_name": "Immunoglobulin heavy constant gamma 4",
  "term_id": "GO:0019731",
  "gene": "UniProtKB:P01861",
  "gene_symbol": "IGHG4"
}